{
  "gene_symbol": "TMPRSS11E",
  "gene_name": "Transmembrane protease serine 11E",
  "term_id": "GO:0008236",
  "gene": "UniProtKB:Q9UL52",
  "term_label": "serine-type peptidase activity"
}